{
  "term_id": "GO:0008047",
  "gene_symbol": "SSBP1",
  "term_label": "enzyme activator activity",
  "gene": "UniProtKB:Q04837",
  "gene_name": "Single-stranded DNA-binding protein, mitochondrial"
}